{
  "term_label": "cytoplasm",
  "term_id": "GO:0005737",
  "gene": "UniProtKB:Q9NXC5",
  "gene_name": "GATOR complex protein MIOS",
  "gene_symbol": "MIOS"
}